guard cell fate commitment [GO:0010377] (biological process) References: PMID:17259259 Definition: The process in which the developmental fate of a cell becomes restricted such that it will develop into a stomatal guard cell. Guard cells are located in the leaf epidermis and pairwise surround stomatal pores, which allow CO2 influx for photosynthetic carbon fixation and water loss via transpiration to the atmosphere. Relationships: is_a cell fate commitment [GO:0045165]; is part of GO:0010052 Also known as: stomatal cell fate commitment